{
  "gene_name": "t-SNARE domain-containing protein 1",
  "gene": "UniProtKB:Q96NA8",
  "term_label": "SNARE complex",
  "gene_symbol": "TSNARE1",
  "term_id": "GO:0031201"
}